{
  "gene": "UniProtKB:P06126",
  "term_label": "external side of plasma membrane",
  "gene_name": "T-cell surface glycoprotein CD1a",
  "gene_symbol": "CD1A",
  "term_id": "GO:0009897"
}